{
  "term_label": "muscle alpha-actinin binding",
  "term_id": "GO:0051371",
  "gene_name": "PDZ and LIM domain protein 7",
  "gene": "UniProtKB:Q9NR12",
  "gene_symbol": "PDLIM7"
}